protein C inhibitor-TMPRSS11E complex [GO:0036025] (CC) Relationships: is a type of serine protease inhibitor complex [GO:0097180] Also known as: PCI-TMPRSS11E complex, SERPINA5-TMPRSS11E complex, plasma serine protease inhibitor-TMPRSS11E complex, protein C inhibitor-transmembrane protease serine 11E complex, serpin A5-TMPRSS11E complex Definition: A heterodimeric protein complex that contains protein C inhibitor (SERPINA5) and transmembrane protease serine 11E (TMPRSS11E); formation of the complex inhibits the serine protease activity of transmembrane protease serine 11E. References: PMID:15328353 Sources: GOC:ans